positive regulation of double-strand break repair via nonhomologous end joining [GO:2001034] (biological process) Definition: Any process that activates or increases the frequency, rate or extent of double-strand break repair via nonhomologous end joining. Also known as: positive regulation of NHEJ Sources: GOC:obol Relationships: is a type of positive regulation of double-strand break repair [GO:2000781]; is a type of regulation of double-strand break repair via nonhomologous end joining [GO:2001032]; positively regulates GO:0006303